retrograde trans-synaptic signaling by neuropeptide [GO:0099082] (biological process) Regulation: regulated by GO:1905432; negatively regulated by negative regulation of retrograde trans-synaptic signaling by neuropeptide [GO:1905433]; positively regulated by positive regulation of retrograde trans-synaptic signaling by neuropeptide [GO:1905434] Subtypes: retrograde trans-synaptic signaling by neuropeptide, modulating synaptic transmission [GO:0099083] Definition: Cell-cell signaling from postsynapse to presynapse, across the synaptic cleft, mediated by a neuropeptide. Relationships: is a type of retrograde trans-synaptic signaling [GO:0098917]; is a type of trans-synaptic signaling by neuropeptide [GO:0099540] References: PMID:19448629 Sources: GOC:PARL, GOC:bf, GOC:dos